chemoattraction of branchiomotor axon [GO:0021792] (biological process) References: PMID:14699587 Sources: GOC:cls, GOC:dgh, GOC:dph, GOC:jid, GO_REF:0000021 Relationships: is a type of chemoattraction of axon [GO:0061642]; is part of branchiomotor neuron axon guidance [GO:0021785] Subtypes: GO:0021788, chemoattraction of branchiomotor neuron axon in branchial arch mesenchyme [GO:0021791] Also known as: positive chemotaxis of branchiomotor axon Definition: The process in which a branchiomotor neuron growth cone is directed to a specific target site in response to an attractive chemical signal. Branchiomotor neurons are located in the hindbrain and innervate branchial arch-derived muscles that control jaw movements, facial expression, the larynx, and the pharynx.